{
  "gene": "UniProtKB:Q86SG3",
  "gene_name": "Deleted in azoospermia protein 4",
  "term_label": "3'-UTR-mediated mRNA stabilization",
  "gene_symbol": "DAZ4",
  "term_id": "GO:0070935"
}